secretion [GO:0046903] (biological process) Sources: GOC:ai Relationships: is_a transport [GO:0006810] Definition: The controlled release of a substance by a cell or a tissue. Subtypes: histamine secretion [GO:0001821], peptide secretion [GO:0002790], body fluid secretion [GO:0007589], canalicular bile acid transport [GO:0015722], icosanoid secretion [GO:0032309], GO:0032940, GO:0032941, acid secretion [GO:0046717], nectar secretion [GO:0071836], apocrine secretion [GO:0160022], surfactant secretion [GO:0160069] Regulation: regulated by regulation of secretion [GO:0051046]; positively regulated by GO:0051047; negatively regulated by negative regulation of secretion [GO:0051048]